{
  "gene_symbol": "MFF",
  "term_label": "mitochondrial outer membrane",
  "gene_name": "Mitochondrial fission factor",
  "gene": "UniProtKB:Q9GZY8",
  "term_id": "GO:0005741"
}